{
  "term_label": "Z disc",
  "gene": "UniProtKB:P17661",
  "term_id": "GO:0030018",
  "gene_name": "Desmin",
  "gene_symbol": "DES"
}